methylarsonate reductase activity [GO:0050610] (molecular function) Sources: EC:1.20.4.2, RHEA:15969 Also known as: MMA(V) reductase activity, glutathione:methylarsonate oxidoreductase activity Definition: Catalysis of the reaction: 2 glutathione + H+ + methylarsonate = glutathione disulfide + H2O + methylarsonous acid. Relationships: is a type of oxidoreductase activity, acting on phosphorus or arsenic in donors, disulfide as acceptor [GO:0030614]